{
  "gene_symbol": "GUSBP11",
  "gene": "UniProtKB:Q6P575",
  "term_id": "UNKNOWN:0002",
  "term_label": "Unknown biological process",
  "gene_name": "Putative inactive beta-glucuronidase protein GUSBP11"
}